{
  "gene_name": "Triggering receptor expressed on myeloid cells 2",
  "gene": "UniProtKB:Q9NZC2",
  "term_label": "plasma membrane",
  "term_id": "GO:0005886",
  "gene_symbol": "TREM2"
}